foraging behavior [GO:0060756] (biological process) Relationships: is a type of behavior [GO:0007610] Regulation: regulated by regulation of foraging behavior [GO:1903368]; negatively regulated by negative regulation of foraging behavior [GO:1903369]; positively regulated by positive regulation of foraging behavior [GO:1903370] Definition: Behavior by which an organism locates food. Sources: GOC:dph, GOC:tb Subtypes: larval foraging behavior [GO:0035177], adult foraging behavior [GO:0060757], foraging behavior by probing substrate [GO:0060758]